protein dimerization activity [GO:0046983] (molecular function) Sources: ISBN:0198506732 Relationships: is a type of protein binding [GO:0005515] Subtypes: protein homodimerization activity [GO:0042803], protein heterodimerization activity [GO:0046982] Definition: The formation of a protein dimer, a macromolecular structure consists of two noncovalently associated identical or nonidentical subunits.